{
  "gene": "UniProtKB:Q9Y3B1",
  "term_id": "GO:0015914",
  "gene_name": "PRELI domain containing protein 3B",
  "term_label": "phospholipid transport",
  "gene_symbol": "PRELID3B"
}